negative regulation of glycine secretion, neurotransmission [GO:1904625] (biological process) Relationships: is a type of GO:0032891; is a type of negative regulation of neurotransmitter secretion [GO:0046929]; is a type of negative regulation of amino acid transport [GO:0051956]; is a type of GO:0060093; is a type of regulation of glycine secretion, neurotransmission [GO:1904624]; negatively regulates glycine secretion, neurotransmission [GO:0061537] Also known as: down regulation of glycine secretion, neurotransmission, down-regulation of glycine secretion, neurotransmission, downregulation of glycine secretion, neurotransmission, inhibition of glycine secretion, neurotransmission References: PMID:22988142 Sources: GOC:TermGenie, GO_REF:0000058 Definition: Any process that stops, prevents or reduces the frequency, rate or extent of glycine secretion, neurotransmission.